{
  "term_id": "UNKNOWN:0003",
  "gene_symbol": "PSG9",
  "term_label": "Unknown cellular component",
  "gene": "UniProtKB:Q00887",
  "gene_name": "Pregnancy-specific beta-1-glycoprotein 9"
}